mitotic cytokinetic process [GO:1902410] (biological process) Definition: Any cytokinetic process that is involved in mitotic cell cycle. Sources: GOC:TermGenie, GOC:mtg_cell_cycle Regulation: regulated by GO:1903436; negatively regulated by negative regulation of mitotic cytokinetic process [GO:1903437]; positively regulated by positive regulation of mitotic cytokinetic process [GO:1903438] Subtypes: primary cell septum biogenesis [GO:0031671], GO:0032130, GO:0061796, midbody abscission [GO:0061952], mitotic division septum assembly [GO:0140278], mitotic actomyosin contractile ring contraction [GO:1902404], assembly of actomyosin apparatus involved in mitotic cytokinesis [GO:1902407], GO:1902408, mitotic cleavage furrow formation [GO:1903673], secondary cell septum biogenesis [GO:1990344], mitotic cleavage furrow ingression [GO:1990386] Relationships: is a type of GO:0032506; is a type of mitotic cell cycle process [GO:1903047]; is part of mitotic cytokinesis [GO:0000281]